{
  "term_id": "GO:0017075",
  "gene": "UniProtKB:Q9UPW8",
  "gene_symbol": "UNC13A",
  "gene_name": "Protein unc-13 homolog A",
  "term_label": "syntaxin-1 binding"
}